{
  "gene_symbol": "SAMHD1",
  "term_label": "dGTP catabolic process",
  "gene_name": "Deoxynucleoside triphosphate triphosphohydrolase SAMHD1",
  "gene": "UniProtKB:Q9Y3Z3",
  "term_id": "GO:0006203"
}